negative regulation of xenobiotic detoxification by transmembrane export across the plasma membrane [GO:1905700] (biological process) Relationships: is a type of negative regulation of transmembrane transport [GO:0034763]; is a type of regulation of xenobiotic detoxification by transmembrane export across the plasma membrane [GO:1905699]; is a type of negative regulation of response to drug [GO:2001024]; negatively regulates xenobiotic detoxification by transmembrane export across the plasma membrane [GO:1990961] Also known as: down regulation of drug transmembrane export, down-regulation of drug transmembrane export, downregulation of drug transmembrane export, inhibition of drug transmembrane export, negative regulation of drug transmembrane export, negative regulation of xenobiotic transmembrane export Definition: Any process that stops, prevents or reduces the frequency, rate or extent of xenobiotic transmembrane export. A xenobiotic is a compound foreign to the organism exposed to it. It may be synthesized by another organism (like ampicilin) or it can be a synthetic chemical. References: PMID:15198509 Sources: GOC:TermGenie, GOC:krc, GO_REF:0000058